TSC1-TSC2 complex [GO:0033596] (cellular component) References: PMID:10585443, PMID:17121544, PMID:9580671 Definition: A protein complex consisting of at least tumerin and hamartin; its formation may regulate hamartin homomultimer formation. The complex acts as a GTPase activating protein (GAP) for the small GTPase (Rheb), and inhibits the TOR signaling pathway. Relationships: is a type of protein-containing complex [GO:0032991]; is part of GO:0005829 Also known as: tuberin-hamartin complex, tuberous sclerosis complex